{
  "gene_symbol": "ITGA10",
  "gene": "UniProtKB:O75578",
  "gene_name": "Integrin alpha-10",
  "term_id": "GO:0038023",
  "term_label": "signaling receptor activity"
}